gamma-aminobutyric acid metabolic process [GO:0009448] (biological process) Note: See also the biological process term 'neurotransmitter metabolic process ; GO:0042133'. Also known as: 4-aminobutanoate metabolic process, 4-aminobutanoate metabolism, 4-aminobutyrate metabolic process, 4-aminobutyrate metabolism, GABA metabolic process, GABA metabolism, gamma-aminobutyric acid metabolism Sources: ISBN:0198506732 Definition: The chemical reactions and pathways involving gamma-aminobutyric acid (GABA, 4-aminobutyrate), an amino acid which acts as a neurotransmitter in some organisms. Relationships: is a type of monocarboxylic acid metabolic process [GO:0032787]; is a type of GO:0170041 Subtypes: gamma-aminobutyric acid biosynthetic process [GO:0009449], GO:0009450